positive regulation of neuron differentiation [GO:0045666] (biological process) Subtypes: positive regulation of mechanoreceptor differentiation [GO:0045633], GO:0046534, positive regulation of glutamatergic neuron differentiation [GO:0120008], positive regulation of spinal cord association neuron differentiation [GO:1902831], GO:1902871, positive regulation of dopaminergic neuron differentiation [GO:1904340], GO:1905081, positive regulation of forebrain neuron differentiation [GO:2000979] Definition: Any process that activates or increases the frequency, rate or extent of neuron differentiation. Sources: GOC:go_curators Relationships: is a type of positive regulation of cell differentiation [GO:0045597]; is a type of GO:0045664; positively regulates neuron differentiation [GO:0030182] Also known as: up regulation of neuron differentiation, up-regulation of neuron differentiation, upregulation of neuron differentiation, activation of neuron differentiation, stimulation of neuron differentiation